preganglionic parasympathetic fiber development [GO:0021783] (BP) Relationships: is a type of system development [GO:0048731]; BFO_0000050 GO:0007417; is part of parasympathetic nervous system development [GO:0048486] Definition: The process whose specific outcome is the progression of a preganglionic parasympathetic fiber over time, from its formation to the mature structure. A preganglionic parasympathetic fiber is a cholinergic axonal fiber projecting from the CNS to a parasympathetic ganglion. Sources: GOC:cjm, GOC:cls, GOC:dgh, GOC:dph, GOC:jid